{
  "term_id": "UNKNOWN:0003",
  "gene_name": "Zinc finger protein 501",
  "gene": "UniProtKB:Q96CX3",
  "gene_symbol": "ZNF501",
  "term_label": "Unknown cellular component"
}